{
  "term_id": "GO:0031647",
  "term_label": "regulation of protein stability",
  "gene_symbol": "USP35",
  "gene_name": "Ubiquitin carboxyl-terminal hydrolase 35",
  "gene": "UniProtKB:Q9P2H5"
}